{
  "gene": "UniProtKB:Q53TQ3",
  "gene_name": "INO80 complex subunit D",
  "gene_symbol": "INO80D",
  "term_label": "nucleus",
  "term_id": "GO:0005634"
}